{
  "term_id": "GO:0005886",
  "gene_name": "Glutamate receptor ionotropic, delta-2",
  "gene": "UniProtKB:O43424",
  "term_label": "plasma membrane",
  "gene_symbol": "GRID2"
}